{
  "term_label": "phosphatidylinositol transfer activity",
  "gene": "UniProtKB:O14523",
  "gene_symbol": "C2CD2L",
  "term_id": "GO:0008526",
  "gene_name": "Phospholipid transfer protein C2CD2L"
}